symmetric division of skeletal muscle satellite stem cell [GO:0098726] (biological process) Definition: The symmetric division of a skeletal muscle satellite stem cell, resulting in two skeletal muscle satellite stem cells. This process is involved in amplification of the pool of these cells. References: PMID:23303905 Relationships: is a type of somatic stem cell division [GO:0048103]; is a type of symmetric stem cell division [GO:0098724]